17-hydroxyprogesterone 21-hydroxylase activity [GO:0103069] (molecular function) Sources: RHEA:50308 Relationships: is a type of GO:0004509 Definition: Catalysis of the reaction: 17alpha-hydroxyprogesterone + O2 + reduced [NADPH--hemoprotein reductase] = 11-deoxycortisol + H+ + H2O + oxidized [NADPH--hemoprotein reductase].